regulation of purine nucleoside transport [GO:0032245] (biological process) Relationships: is a type of GO:0032242 Sources: GOC:mah Definition: Any process that modulates the frequency, rate or extent of the directed movement of a purine nucleoside into, out of or within a cell, or between cells, by means of some agent such as a transporter or pore. Subtypes: negative regulation of purine nucleoside transport [GO:0032247], positive regulation of purine nucleoside transport [GO:0032248], GO:0032249, GO:0035341